{
  "gene_name": "R-spondin-3",
  "term_id": "GO:0005109",
  "term_label": "frizzled binding",
  "gene_symbol": "RSPO3",
  "gene": "UniProtKB:Q9BXY4"
}